actin rod [GO:0031002] (cellular component) Subtypes: cofilin-actin rod [GO:0090732] Definition: A cellular structure consisting of parallel, hexagonally arranged actin tubules, comprising filamentous actin and associated proteins. Actin rod structures are found in diverse organisms, having been observed in spores of Dictyostelium discoideum, Drosophila melanogaster oocytes, as well as in numerous animal cells under stress conditions. Relationships: is a type of actin filament bundle [GO:0032432] References: PMID:11858703, PMID:19459188, PMID:22623727, PMID:24813767, PMID:27535426, PMID:7820870 Sources: GOC:kp, GOC:krc